{
  "term_label": "cytosolic large ribosomal subunit",
  "gene": "UniProtKB:Q9Y3U8",
  "gene_name": "Large ribosomal subunit protein eL36",
  "gene_symbol": "RPL36",
  "term_id": "GO:0022625"
}